{
  "gene_name": "Villin-like protein",
  "term_label": "phosphatidylinositol-4,5-bisphosphate binding",
  "term_id": "GO:0005546",
  "gene": "UniProtKB:O15195",
  "gene_symbol": "VILL"
}